{
  "term_id": "GO:0022625",
  "gene_symbol": "RPL18",
  "gene": "UniProtKB:Q07020",
  "term_label": "cytosolic large ribosomal subunit",
  "gene_name": "Large ribosomal subunit protein eL18"
}